{
  "term_label": "cytoplasmic vesicle",
  "gene_symbol": "RNF157",
  "term_id": "GO:0031410",
  "gene": "UniProtKB:Q96PX1",
  "gene_name": "E3 ubiquitin ligase RNF157"
}